{
  "term_id": "GO:0042734",
  "term_label": "presynaptic membrane",
  "gene_symbol": "RIMS2",
  "gene": "UniProtKB:Q9UQ26",
  "gene_name": "Regulating synaptic membrane exocytosis protein 2"
}